intramolecular lyase activity [GO:0016872] (molecular function) Definition: The catalysis of certain rearrangements of a molecule to break or form a ring. Subtypes: inositol-3-phosphate synthase activity [GO:0004512], GO:0009905, muconate cycloisomerase activity [GO:0018849], chloromuconate cycloisomerase activity [GO:0018850], alpha-pinene-oxide decyclase activity [GO:0018851], dichloromuconate cycloisomerase activity [GO:0018852], GO:0035439, chalcone isomerase activity [GO:0045430], 3-carboxy-cis,cis-muconate cycloisomerase activity [GO:0047472], carboxy-cis,cis-muconate cyclase activity [GO:0047768], cycloeucalenol cycloisomerase activity [GO:0047793], GO:0047926, tetrahydroxypteridine cycloisomerase activity [GO:0050329], copalyl diphosphate synthase activity [GO:0050559], GO:0051498, kolavenyl diphosphate synthase activity [GO:0106242] Relationships: is a type of isomerase activity [GO:0016853] Sources: GOC:jl